{
  "gene": "UniProtKB:Q9H607",
  "term_label": "bicellular tight junction assembly",
  "term_id": "GO:0070830",
  "gene_symbol": "OCEL1",
  "gene_name": "Occludin_ELL domain-containing protein 1"
}